cardioblast cell midline fusion [GO:0003317] (biological process) Relationships: is_a homotypic cell-cell adhesion [GO:0034109]; is a type of cell adhesion involved in heart morphogenesis [GO:0061343]; is part of heart rudiment formation [GO:0003315] Also known as: cardiac progenitor cell midline fusion Definition: The attachment of cardiac progenitor cells to one another that contributes to the formation of the heart rudiment. Sources: GOC:mtg_heart